translational elongation [GO:0006414] (biological process) Subtypes: GO:0002182, GO:0006451, translational frameshifting [GO:0006452], mitochondrial translational elongation [GO:0070125], trans-translation [GO:0070929], rescue of stalled ribosome [GO:0072344] Sources: GOC:ems Definition: The successive addition of amino acid residues to a nascent polypeptide chain during protein biosynthesis. Regulation: regulated by regulation of translational elongation [GO:0006448]; negatively regulated by negative regulation of translational elongation [GO:0045900]; positively regulated by positive regulation of translational elongation [GO:0045901] Relationships: is a type of macromolecule biosynthetic process [GO:0009059]; is part of GO:0006412 Also known as: protein synthesis elongation, translation elongation